{
  "gene_name": "Coiled-coil domain-containing protein 34",
  "gene_symbol": "CCDC34",
  "term_label": "Unknown molecular function",
  "term_id": "UNKNOWN:0001",
  "gene": "UniProtKB:Q96HJ3"
}